{
  "term_id": "GO:0007409",
  "gene_symbol": "FAT4",
  "gene_name": "Protocadherin Fat 4",
  "term_label": "axonogenesis",
  "gene": "UniProtKB:Q6V0I7"
}